{
  "term_label": "pyruvate transmembrane transporter activity",
  "gene": "UniProtKB:O95563",
  "gene_symbol": "MPC2",
  "gene_name": "Mitochondrial pyruvate carrier 2",
  "term_id": "GO:0050833"
}